new spindle pole body SIN signaling complex [GO:0160067] (cellular component) Also known as: new spindle pole body SIN signalling complex Relationships: is_a SIN/MEN signaling complex [GO:0160065] Definition: A SIN signaling complex associated with the new mitotic spindle pole body during anaphase and characterized by the presence activated (GTP bound) GTPase (Spg1 in fission yeast) to activate SIN signaling. References: PMID:21131906